{
  "term_label": "cytoplasm",
  "gene": "UniProtKB:P49137",
  "term_id": "GO:0005737",
  "gene_symbol": "MAPKAPK2",
  "gene_name": "MAP kinase-activated protein kinase 2"
}